{
  "term_id": "GO:0002430",
  "term_label": "complement receptor mediated signaling pathway",
  "gene": "UniProtKB:Q16581",
  "gene_name": "C3a anaphylatoxin chemotactic receptor",
  "gene_symbol": "C3AR1"
}